regulation of embryo sac central cell differentiation [GO:0045691] (biological process) Subtypes: negative regulation of embryo sac central cell differentiation [GO:0045692], positive regulation of embryo sac central cell differentiation [GO:0045693] Also known as: regulation of female gametophyte central cell differentiation Sources: GOC:go_curators, GOC:mtg_plant Relationships: is a type of GO:0045595; is a type of regulation of multicellular organismal development [GO:2000026]; regulates embryo sac central cell differentiation [GO:0009559] Definition: Any process that modulates the frequency, rate or extent of female gametophyte central cell differentiation.